{
  "gene_symbol": "ALDOC",
  "gene_name": "Fructose-bisphosphate aldolase C",
  "term_id": "GO:0030388",
  "term_label": "fructose 1,6-bisphosphate metabolic process",
  "gene": "UniProtKB:P09972"
}